{
  "gene_name": "Adenylosuccinate lyase",
  "gene": "UniProtKB:P30566",
  "term_label": "'de novo' AMP biosynthetic process",
  "gene_symbol": "ADSL",
  "term_id": "GO:0044208"
}